male-female gamete recognition during double fertilization forming a zygote and endosperm [GO:0080173] (biological process) References: PMID:21123745 Also known as: gamete recognition, male-female gamete recognition Relationships: is a type of cell-cell recognition [GO:0009988]; is a type of cellular process involved in reproduction in multicellular organism [GO:0022412]; is part of GO:0061936 Definition: The initial contact step made between the male gamete and the female gamete during double fertilization forming a zygote and endosperm. An example can be found in Arabidopsis thaliana.